AGA codon-amino acid adaptor activity [GO:0033447] (molecular function) Definition: A triplet codon-amino acid adaptor activity that recognizes an AGA codon. Sources: GOC:mah Also known as: arginine tRNA Note: Note that in the standard genetic code, AGA codes for arginine. Relationships: is a type of triplet codon-amino acid adaptor activity [GO:0030533]